{
  "term_id": "GO:0030425",
  "gene_symbol": "EPHA4",
  "term_label": "dendrite",
  "gene": "UniProtKB:P54764",
  "gene_name": "Ephrin type-A receptor 4"
}